metal cation:monoatomic cation antiporter activity [GO:0140828] (MF) Subtypes: calcium:monoatomic cation antiporter activity [GO:0015368], solute:potassium antiporter activity [GO:0022821], metal cation:proton antiporter activity [GO:0051139], magnesium:sodium antiporter activity [GO:0061768], sodium,bicarbonate:chloride antiporter activity [GO:0140892] Also known as: solute:metal cation antiporter activity Definition: Enables the transfer of a solute or solutes from one side of a membrane to the other according to the reaction: solute(out) + Na+(in) = solute(in) + Na+(out). Sources: GOC:pg Relationships: is a type of antiporter activity [GO:0015297]; is_a metal ion transmembrane transporter activity [GO:0046873]